{
  "gene_name": "Nuclear protein localization protein 4 homolog",
  "term_label": "ubiquitin binding",
  "gene": "UniProtKB:Q8TAT6",
  "gene_symbol": "NPLOC4",
  "term_id": "GO:0043130"
}